{
  "gene_name": "Ig-like V-type domain-containing protein FAM187A",
  "gene_symbol": "FAM187A",
  "term_id": "UNKNOWN:0001",
  "term_label": "Unknown molecular function",
  "gene": "UniProtKB:A6NFU0"
}